histone acetyltransferase complex [GO:0000123] (cellular component) Definition: A protein complex that possesses histone acetyltransferase activity. Sources: GOC:mah Also known as: histone acetylase complex Note: Note that this term represents a protein complex, not a function; the activity possessed by this complex is mentioned in the definition for the purpose of describing and distinguishing the complex. The function of this complex is represented by the molecular function term 'histone acetyltransferase activity ; GO:0004402'. Relationships: is a type of protein acetyltransferase complex [GO:0031248]; is part of GO:0000785 Subtypes: GO:0070461, H3 histone acetyltransferase complex [GO:0070775], H4 histone acetyltransferase complex [GO:1902562]